L-lysine catabolic process to acetyl-CoA via 5-aminopentanamide [GO:0033513] (biological process) Also known as: L-lysine breakdown to acetyl-CoA via 5-aminopentanamide, L-lysine degradation to acetyl-CoA via 5-aminopentanamide Definition: The chemical reactions and pathways resulting in the breakdown of L-lysine into other compounds, including acetyl-CoA, via the intermediate 5-aminopentanamide. Sources: GOC:mah, MetaCyc:PWY-5280 Relationships: is a type of L-lysine catabolic process to acetyl-CoA [GO:0019474]